beta-1,4-mannosylglycoprotein 4-beta-N-acetylglucosaminyltransferase activity [GO:0003830] (molecular function) Definition: Catalysis of the reaction: UDP-N-acetyl-D-glucosamine + beta-D-mannosyl-R = UDP + 4-(N-acetyl-beta-D-glucosaminyl)-beta-D-mannosyl-R. Sources: EC:2.4.1.144 Also known as: GnTIII activity, N-acetylglucosaminyltransferase III activity, N-glycosyl-oligosaccharide-glycoprotein N-acetylglucosaminyltransferase III activity, UDP-N-acetyl-D-glucosamine:beta-D-mannosyl-glycoprotein 4-beta-N-acetyl-D-glucosaminyltransferase activity, beta-1,4-mannosyl-glycoprotein 4-beta-N-acetylglucosaminyltransferase activity, beta-1,4-mannosyl-glycoprotein beta-1,4-N-acetylglucosaminyltransferase activity, uridine diphosphoacetylglucosamine-glycopeptide beta-4-acetylglucosaminyltransferase III activity, uridine diphosphoacetylglucosamine-glycopeptide beta4-acetylglucosaminyltransferase III Relationships: is a type of acetylglucosaminyltransferase activity [GO:0008375]; is a type of catalytic activity, acting on a glycoprotein [GO:0140103]